bis(2-ethylhexyl)phthalate esterase activity [GO:0047709] (molecular function) Sources: EC:3.1.1.60, RHEA:15529 Relationships: is a type of carboxylic ester hydrolase activity [GO:0052689] Definition: Catalysis of the reaction: bis(2-ethylhexyl)phthalate + H2O = 2-ethylhexan-1-ol + 2-ethylhexyl phthalate + H+. Also known as: DEHP esterase activity, bis(2-ethylhexyl)phthalate acylhydrolase activity